{
  "gene_symbol": "GVQW3",
  "term_id": "UNKNOWN:0002",
  "term_label": "Unknown biological process",
  "gene": "UniProtKB:Q3ZCU0",
  "gene_name": "Protein GVQW3"
}